{
  "gene": "UniProtKB:Q9NZU5",
  "term_label": "Unknown biological process",
  "term_id": "UNKNOWN:0002",
  "gene_symbol": "LMCD1",
  "gene_name": "LIM and cysteine-rich domains protein 1"
}